prostaglandin-I synthase activity [GO:0008116] (molecular function) Relationships: is_a intramolecular oxidoreductase activity [GO:0016860] Also known as: cytochrome P450 CYP8A1, (5Z,13E)-(15S)-9alpha,11alpha-epidioxy-15-hydroxyprosta-5,13-dienoate 6-isomerase activity, PGI(2) synthase activity, PGI(2) synthetase activity, PGI2 synthase activity, PGI2 synthetase activity, prostacyclin synthase activity, prostacycline synthetase activity, prostagladin I2 synthetase activity Definition: Catalysis of the reaction: prostaglandin H(2) = prostaglandin I(2). Sources: EC:5.3.99.4, RHEA:23580